{
  "gene_symbol": "MYLK3",
  "term_label": "cardiac myofibril assembly",
  "term_id": "GO:0055003",
  "gene": "UniProtKB:Q32MK0",
  "gene_name": "Myosin light chain kinase 3"
}